ER to Golgi transport vesicle membrane [GO:0012507] (CC) Sources: GOC:ai, GOC:ascb_2009, GOC:dph, GOC:tb Also known as: COPII coated vesicle membrane, ER to Golgi constitutive secretory pathway transport vesicle membrane, ER-Golgi transport vesicle membrane, endoplasmic reticulum to Golgi transport vesicle membrane, endoplasmic reticulum-Golgi transport vesicle membrane Relationships: is a type of GO:0030658; is a type of coated vesicle membrane [GO:0030662]; is part of COPII-coated ER to Golgi transport vesicle [GO:0030134] Definition: The lipid bilayer surrounding a vesicle transporting substances from the endoplasmic reticulum to the Golgi.